{
  "term_label": "nucleolus",
  "gene_name": "WD repeat-containing protein 46",
  "gene_symbol": "WDR46",
  "gene": "UniProtKB:O15213",
  "term_id": "GO:0005730"
}